{
  "term_label": "protein ubiquitination",
  "gene_name": "E3 ubiquitin-protein ligase RNF183",
  "term_id": "GO:0016567",
  "gene_symbol": "RNF183",
  "gene": "UniProtKB:Q96D59"
}